{
  "term_id": "UNKNOWN:0003",
  "gene_name": "Putative rhophilin-2-like protein RHPN2P1",
  "gene_symbol": "RHPN2P1",
  "gene": "UniProtKB:A8MT19",
  "term_label": "Unknown cellular component"
}